{
  "gene": "UniProtKB:Q08ER8",
  "gene_name": "Zinc finger protein 543",
  "gene_symbol": "ZNF543",
  "term_id": "GO:0000978",
  "term_label": "RNA polymerase II cis-regulatory region sequence-specific DNA binding"
}